{
  "term_label": "Unknown molecular function",
  "gene": "UniProtKB:Q969P5",
  "gene_name": "F-box only protein 32",
  "gene_symbol": "FBXO32",
  "term_id": "UNKNOWN:0001"
}